tongue morphogenesis [GO:0043587] (biological process) Definition: The process in which the anatomical structures of the tongue are generated and organized. The tongue is the movable, muscular organ on the floor of the mouth of most vertebrates, in man other mammals is the principal organ of taste, aids in the prehension of food, in swallowing, and in modifying the voice as in speech. Sources: GOC:jl, UBERON:0001723 Also known as: lingua morphogenesis, glossa morphogenesis Relationships: is a type of sensory organ morphogenesis [GO:0090596]; is part of tongue development [GO:0043586]